{
  "gene_symbol": "KBTBD12",
  "term_label": "ubiquitin-like ligase-substrate adaptor activity",
  "gene_name": "Kelch repeat and BTB domain-containing protein 12",
  "term_id": "GO:1990756",
  "gene": "UniProtKB:Q3ZCT8"
}